interleukin-25 binding [GO:0045511] (molecular function) Definition: Binding to interleukin-25. Sources: GOC:go_curators Also known as: IL-25 binding Relationships: is a type of interleukin-17 binding [GO:0019975]